{
  "gene": "UniProtKB:Q9NY72",
  "term_label": "ventricular cardiac muscle cell action potential",
  "term_id": "GO:0086005",
  "gene_name": "Sodium channel subunit beta-3",
  "gene_symbol": "SCN3B"
}